{
  "term_label": "nucleus",
  "gene_name": "Aryl hydrocarbon receptor nuclear translocator 2",
  "term_id": "GO:0005634",
  "gene": "UniProtKB:Q9HBZ2",
  "gene_symbol": "ARNT2"
}